{
  "term_id": "GO:0005789",
  "term_label": "endoplasmic reticulum membrane",
  "gene": "UniProtKB:Q9H1N7",
  "gene_symbol": "SLC35B3",
  "gene_name": "Adenosine 3'-phospho 5'-phosphosulfate transporter 2"
}